{
  "term_id": "GO:0005737",
  "gene_symbol": "KLHL23",
  "gene": "UniProtKB:Q8NBE8",
  "term_label": "cytoplasm",
  "gene_name": "Kelch-like protein 23"
}